{
  "gene": "UniProtKB:Q7Z2T5",
  "term_label": "tRNA (guanine) methyltransferase activity",
  "gene_symbol": "TRMT1L",
  "gene_name": "TRMT1-like protein",
  "term_id": "GO:0016423"
}